{
  "term_label": "plasma membrane",
  "gene_name": "Neuronal acetylcholine receptor subunit beta-2",
  "gene": "UniProtKB:P17787",
  "term_id": "GO:0005886",
  "gene_symbol": "CHRNB2"
}